{
  "gene": "UniProtKB:P11021",
  "gene_symbol": "HSPA5",
  "term_label": "endoplasmic reticulum chaperone complex",
  "term_id": "GO:0034663",
  "gene_name": "Endoplasmic reticulum chaperone BiP"
}